{
  "gene": "UniProtKB:P02656",
  "term_id": "GO:0010987",
  "term_label": "negative regulation of high-density lipoprotein particle clearance",
  "gene_name": "Apolipoprotein C-III",
  "gene_symbol": "APOC3"
}